{
  "gene": "UniProtKB:P24557",
  "gene_symbol": "TBXAS1",
  "term_label": "Unknown biological process",
  "gene_name": "Thromboxane-A synthase",
  "term_id": "UNKNOWN:0002"
}